prophase [GO:0051324] (biological process) Definition: The cell cycle phase which is the first stage of M phase of meiosis and mitosis and during which chromosomes condense and the two daughter centrioles and their asters migrate toward the poles of the cell. Subtypes: mitotic prophase [GO:0000088], meiotic prophase I [GO:0007128], meiotic prophase II [GO:0007136] Relationships: is_a cell cycle phase [GO:0022403]; is part of M phase [GO:0000279] Sources: GOC:mtg_cell_cycle Note: Note that this term should not be used for direct annotation. If you are trying to make an annotation to x phase, it is likely that the correct annotation is 'regulation of x/y phase transition' or to a process which occurs during the reported phase (i.e mitotic DNA replication for mitotic S-phase). To capture the phase when a specific location or process is observed, the phase term can be used in an annotation extension (PMID:24885854) applied to a cellular component term (with the relation exists_during) or a biological process term (with the relation happens_during).